{
  "gene": "UniProtKB:O15457",
  "gene_symbol": "MSH4",
  "term_label": "double-stranded DNA binding",
  "term_id": "GO:0003690",
  "gene_name": "MutS protein homolog 4"
}